{
  "gene": "UniProtKB:P01911",
  "term_id": "GO:0050778",
  "gene_name": "HLA class II histocompatibility antigen, DRB1 beta chain",
  "gene_symbol": "HLA-DRB1",
  "term_label": "positive regulation of immune response"
}